{
  "term_id": "GO:0070006",
  "gene_name": "Aminopeptidase N",
  "gene": "UniProtKB:P15144",
  "gene_symbol": "ANPEP",
  "term_label": "metalloaminopeptidase activity"
}